{
  "gene": "UniProtKB:Q9Y366",
  "gene_name": "Intraflagellar transport protein 52 homolog",
  "term_label": "intraciliary transport particle B",
  "gene_symbol": "IFT52",
  "term_id": "GO:0030992"
}